{
  "gene": "UniProtKB:P40425",
  "term_label": "neuron development",
  "gene_symbol": "PBX2",
  "term_id": "GO:0048666",
  "gene_name": "Pre-B-cell leukemia transcription factor 2"
}